{
  "gene": "UniProtKB:P11274",
  "gene_symbol": "BCR",
  "term_id": "UNKNOWN:0001",
  "gene_name": "Breakpoint cluster region protein",
  "term_label": "Unknown molecular function"
}